{
  "gene_name": "Netrin receptor DCC",
  "term_label": "axon guidance",
  "gene": "UniProtKB:P43146",
  "gene_symbol": "DCC",
  "term_id": "GO:0007411"
}